{
  "gene": "UniProtKB:Q30201",
  "term_label": "response to iron ion starvation",
  "term_id": "GO:1990641",
  "gene_symbol": "HFE",
  "gene_name": "Hereditary hemochromatosis protein"
}